EMC complex [GO:0072546] (cellular component) Note: Note that this complex used to be thought to be involved in ER-mitochondrial membrane tethering, which is required to facilitate lipid transfer from the ER to the mitochondrial membrane, but newer findings show that this was incorrect. References: PMID:29242231, PMID:30415835, PMID:32459176 Also known as: ER membrane protein complex, endoplasmic reticulum membrane protein complex Relationships: is a type of membrane protein complex [GO:0098796]; is a type of GO:0140534; BFO_0000050 GO:0005789 Definition: A transmembrane protein complex located in the endoplasmic reticulum (ER) involved in the insertion of newly synthesized proteins in the membrane of the ER. In S. cerevisiae, it has six members: EMC1, EMC2, AIM27, EMC4, KRE27, and EMC6.